positive regulation of lamellipodium assembly [GO:0010592] (BP) Relationships: is a type of regulation of lamellipodium assembly [GO:0010591]; is_a positive regulation of plasma membrane bounded cell projection assembly [GO:0120034]; is a type of positive regulation of lamellipodium organization [GO:1902745]; positively regulates GO:0030032 Definition: Any process that increases the rate, frequency or extent of the formation of a lamellipodium, a thin sheetlike extension of the surface of a migrating cell. Sources: GOC:dph, GOC:tb Also known as: positive regulation of lamellipodium biogenesis